{
  "gene_name": "Neuroligin-4, X-linked",
  "term_id": "UNKNOWN:0001",
  "gene_symbol": "NLGN4X",
  "gene": "UniProtKB:Q8N0W4",
  "term_label": "Unknown molecular function"
}